negative regulation of granulosa cell apoptotic process [GO:1904709] (biological process) Definition: Any process that stops, prevents or reduces the frequency, rate or extent of granulosa cell apoptotic process. References: PMID:19208546 Sources: GOC:TermGenie, GO_REF:0000058 Also known as: down regulation of granulosa cell apoptotic process, down regulation of granulosa cell of ovary apoptotic process, down-regulation of granulosa cell apoptotic process, down-regulation of granulosa cell of ovary apoptotic process, downregulation of granulosa cell apoptotic process, downregulation of granulosa cell of ovary apoptotic process, negative regulation of granulosa cell of ovary apoptotic process, down regulation of granulosa cell apoptosis, down regulation of granulosa cell of ovary apoptosis, down-regulation of granulosa cell apoptosis, down-regulation of granulosa cell of ovary apoptosis, downregulation of granulosa cell apoptosis, downregulation of granulosa cell of ovary apoptosis, inhibition of granulosa cell apoptosis, inhibition of granulosa cell apoptotic process, inhibition of granulosa cell of ovary apoptosis, inhibition of granulosa cell of ovary apoptotic process, negative regulation of granulosa cell apoptosis, negative regulation of granulosa cell of ovary apoptosis Relationships: is a type of GO:1904036; is a type of GO:1904708; negatively regulates GO:1904700